{
  "gene_symbol": "KCNH6",
  "gene_name": "Potassium voltage-gated channel subfamily H member 6",
  "term_id": "GO:0086013",
  "term_label": "membrane repolarization during cardiac muscle cell action potential",
  "gene": "UniProtKB:Q9H252"
}